negative regulation of ubiquitin-dependent protein catabolic process [GO:2000059] (biological process) Subtypes: negative regulation of proteasomal ubiquitin-dependent protein catabolic process [GO:0032435] Definition: Any process that stops, prevents, or reduces the frequency, rate or extent of ubiquitin-dependent protein catabolic process. Also known as: negative regulation of protein degradation tagging activity, negative regulation of protein ubiquitination during ubiquitin-dependent protein breakdown, negative regulation of protein ubiquitination during ubiquitin-dependent protein catabolic process, negative regulation of protein ubiquitination during ubiquitin-dependent protein catabolism, negative regulation of protein ubiquitination during ubiquitin-dependent protein degradation, negative regulation of protein ubiquitination involved in ubiquitin-dependent protein catabolic process, negative regulation of protein ubiquitinylation during ubiquitin-dependent protein catabolic process, negative regulation of protein ubiquitinylation during ubiquitin-dependent protein catabolism, negative regulation of protein ubiquitylation during ubiquitin-dependent protein catabolic process, negative regulation of protein ubiquitylation during ubiquitin-dependent protein catabolism Relationships: is a type of negative regulation of catabolic process [GO:0009895]; is a type of negative regulation of proteolysis involved in protein catabolic process [GO:1903051]; is a type of GO:2000058; RO_0002212 ubiquitin-dependent protein catabolic process [GO:0006511] Sources: GOC:BHF